microspike assembly [GO:0030035] (BP) Definition: Formation of a microspike, a dynamic, actin-rich projection extending from the surface of a migrating animal cell. Relationships: is a type of plasma membrane bounded cell projection assembly [GO:0120031] Also known as: microspike biosynthesis, microspike formation, microspike biogenesis Note: Although in some literature 'microspike' and 'filopodium' are used synonymously, in GO microspike refers to a cell projection that is distinct from a filopodium. For the assembly of filopodia, use 'filopodium assembly ; GO:0046847'. References: PMID:11429692, PMID:12153987, PMID:19095735 Sources: ISBN:0815316194